{
  "term_label": "positive regulation of receptor signaling pathway via JAK-STAT",
  "term_id": "GO:0046427",
  "gene_symbol": "GHR",
  "gene": "UniProtKB:P10912",
  "gene_name": "Growth hormone receptor"
}